UMP metabolic process [GO:0046049] (biological process) Definition: The chemical reactions and pathways involving UMP, uridine monophosphate. Sources: GOC:go_curators Also known as: UMP metabolism Relationships: is a type of pyrimidine ribonucleoside monophosphate metabolic process [GO:0009173]; is a type of GO:0009218 Subtypes: UMP biosynthetic process [GO:0006222], GO:0046050